{
  "gene": "UniProtKB:O75385",
  "term_id": "GO:0048671",
  "gene_name": "Serine_threonine-protein kinase ULK1",
  "term_label": "negative regulation of collateral sprouting",
  "gene_symbol": "ULK1"
}